{
  "gene_symbol": "KCNK16",
  "term_label": "potassium ion transmembrane transport",
  "term_id": "GO:0071805",
  "gene_name": "Potassium channel subfamily K member 16",
  "gene": "UniProtKB:Q96T55"
}